{
  "gene_symbol": "DNAH14",
  "gene": "UniProtKB:Q0VDD8",
  "term_id": "GO:0030286",
  "term_label": "dynein complex",
  "gene_name": "Dynein axonemal heavy chain 14"
}